{
  "term_id": "GO:0007338",
  "gene_name": "Coiled-coil domain-containing protein 136",
  "gene": "UniProtKB:Q96JN2",
  "gene_symbol": "CCDC136",
  "term_label": "single fertilization"
}